{
  "term_id": "UNKNOWN:0001",
  "term_label": "Unknown molecular function",
  "gene_name": "Vang-like protein 2",
  "gene": "UniProtKB:Q9ULK5",
  "gene_symbol": "VANGL2"
}